{
  "term_id": "UNKNOWN:0003",
  "term_label": "Unknown cellular component",
  "gene": "UniProtKB:A1YPR0",
  "gene_name": "Zinc finger and BTB domain-containing protein 7C",
  "gene_symbol": "ZBTB7C"
}